{
  "term_id": "GO:0016567",
  "term_label": "protein ubiquitination",
  "gene_name": "DDB1- and CUL4-associated factor 15",
  "gene_symbol": "DCAF15",
  "gene": "UniProtKB:Q66K64"
}